positive regulation of synaptic transmission, dopaminergic [GO:0032226] (biological process) Definition: Any process that activates, maintains or increases the frequency, rate or extent of dopaminergic synaptic transmission, the process of communication from a neuron to another neuron across a synapse using the neurotransmitter dopamine. Sources: GOC:mah Also known as: up regulation of synaptic transmission, dopaminergic, up-regulation of synaptic transmission, dopaminergic, upregulation of synaptic transmission, dopaminergic, activation of synaptic transmission, dopaminergic, stimulation of synaptic transmission, dopaminergic Relationships: is a type of regulation of synaptic transmission, dopaminergic [GO:0032225]; is a type of positive regulation of synaptic transmission [GO:0050806]; positively regulates synaptic transmission, dopaminergic [GO:0001963]